{
  "gene": "UniProtKB:P98172",
  "gene_name": "Ephrin-B1",
  "term_label": "plasma membrane",
  "gene_symbol": "EFNB1",
  "term_id": "GO:0005886"
}